{
  "term_id": "UNKNOWN:0002",
  "gene": "UniProtKB:Q9BTY7",
  "term_label": "Unknown biological process",
  "gene_symbol": "HGH1",
  "gene_name": "Protein HGH1 homolog"
}